{
  "term_label": "cytokine receptor activity",
  "gene_name": "Leukemia inhibitory factor receptor",
  "term_id": "GO:0004896",
  "gene": "UniProtKB:P42702",
  "gene_symbol": "LIFR"
}